{
  "gene": "UniProtKB:Q16658",
  "term_label": "actin filament binding",
  "gene_name": "Fascin",
  "term_id": "GO:0051015",
  "gene_symbol": "FSCN1"
}